{
  "gene": "UniProtKB:Q5VST9",
  "gene_symbol": "OBSCN",
  "gene_name": "Obscurin",
  "term_label": "Z disc",
  "term_id": "GO:0030018"
}